RNA-templated viral transcription [GO:0039696] (biological process) Relationships: is a type of viral transcription [GO:0019083] Sources: GOC:bf, GOC:jl Subtypes: negative stranded viral RNA transcription [GO:0039697] Definition: A transcription process that uses viral RNA as a template.